{
  "gene_symbol": "LEG1",
  "gene_name": "Protein LEG1 homolog",
  "term_id": "GO:0005615",
  "term_label": "extracellular space",
  "gene": "UniProtKB:Q6P5S2"
}